{
  "term_id": "GO:0007165",
  "gene": "UniProtKB:Q9H0C8",
  "gene_symbol": "ILKAP",
  "term_label": "signal transduction",
  "gene_name": "Integrin-linked kinase-associated serine_threonine phosphatase 2C"
}